{
  "term_id": "GO:0007218",
  "gene_name": "Prolactin-releasing peptide receptor",
  "term_label": "neuropeptide signaling pathway",
  "gene": "UniProtKB:P49683",
  "gene_symbol": "PRLHR"
}